{
  "gene_symbol": "ZSCAN5A",
  "term_label": "Unknown cellular component",
  "term_id": "UNKNOWN:0003",
  "gene_name": "Zinc finger and SCAN domain-containing protein 5A",
  "gene": "UniProtKB:Q9BUG6"
}